response to glycine [GO:1905429] (biological process) Relationships: is a type of GO:0043200; is a type of response to nitrogen compound [GO:1901698]; is a type of response to oxygen-containing compound [GO:1901700] Also known as: response to Gly, response to aminoacetic acid, response to aminoethanoic acid, response to glycin Definition: Any process that results in a change in state or activity of a cell or an organism (in terms of movement, secretion, enzyme production, gene expression, etc.) as a result of a glycine stimulus. References: PMID:18984164 Sources: GOC:TermGenie, GO_REF:0000071 Subtypes: cellular response to glycine [GO:1905430]